{
  "term_label": "regulation of transcription by RNA polymerase II",
  "gene_symbol": "ZNF44",
  "gene_name": "Zinc finger protein 44",
  "term_id": "GO:0006357",
  "gene": "UniProtKB:P15621"
}